{
  "term_label": "aminophospholipid flippase activity",
  "term_id": "GO:0015247",
  "gene_name": "Cell cycle control protein 50B",
  "gene": "UniProtKB:Q3MIR4",
  "gene_symbol": "TMEM30B"
}